{
  "gene": "UniProtKB:O75293",
  "term_id": "GO:0005634",
  "gene_name": "Growth arrest and DNA damage-inducible protein GADD45 beta",
  "gene_symbol": "GADD45B",
  "term_label": "nucleus"
}